photosynthetic phosphorylation [GO:0009777] (biological process) Definition: Any metabolic process in which photosynthetic organisms use light energy to convert ADP to ATP without the concomitant reduction of dioxygen (O2) to water that occurs in phosphorylation. Also known as: photosynthetic ATP synthesis Subtypes: cyclic photosynthetic phosphorylation [GO:0009778], noncyclic photosynthetic phosphorylation [GO:0009779] Sources: ISBN:0198547684 Relationships: is a type of phosphorylation [GO:0016310]; BFO_0000050 photosynthesis, light reaction [GO:0019684]; BFO_0000051 GO:0015986